{
  "term_label": "tRNA methyltransferase activity",
  "gene": "UniProtKB:Q32P41",
  "gene_symbol": "TRMT5",
  "gene_name": "tRNA (guanine(37)-N1)-methyltransferase",
  "term_id": "GO:0008175"
}